{
  "term_label": "RNA polymerase II transcription regulator complex",
  "gene": "UniProtKB:Q99929",
  "gene_symbol": "ASCL2",
  "gene_name": "Achaete-scute homolog 2",
  "term_id": "GO:0090575"
}